{
  "term_id": "UNKNOWN:0002",
  "term_label": "Unknown biological process",
  "gene_name": "Proline-rich protein 20B",
  "gene": "UniProtKB:P86481",
  "gene_symbol": "PRR20B"
}